{
  "gene_symbol": "PHKG1",
  "term_id": "GO:0007165",
  "gene_name": "Phosphorylase b kinase gamma catalytic chain, skeletal muscle_heart isoform",
  "gene": "UniProtKB:Q16816",
  "term_label": "signal transduction"
}